alpha3-beta1 integrin-tissue transglutaminase complex [GO:0071092] (cellular component) Relationships: is a type of plasma membrane protein complex [GO:0098797]; is a type of catalytic complex [GO:1902494] References: PMID:10684262 Also known as: ITGA3-ITGB1-TGM2 complex Definition: A protein complex that consists of an alpha3-beta1 integrin complex bound to tissue transglutaminase.